{
  "term_id": "GO:0038023",
  "gene_symbol": "ADIPOR1",
  "gene": "UniProtKB:Q96A54",
  "gene_name": "Adiponectin receptor protein 1",
  "term_label": "signaling receptor activity"
}